{
  "gene_name": "Psoriasis susceptibility 1 candidate gene 1 protein",
  "gene": "UniProtKB:Q9UIG5",
  "gene_symbol": "PSORS1C1",
  "term_id": "UNKNOWN:0002",
  "term_label": "Unknown biological process"
}